{
  "gene_name": "Novel acetylcholine receptor chaperone",
  "term_id": "GO:2000010",
  "term_label": "positive regulation of protein localization to cell surface",
  "gene_symbol": "TMEM35A",
  "gene": "UniProtKB:Q53FP2"
}